olivetolic acid biosynthetic process [GO:1901697] (biological process) Definition: The chemical reactions and pathways resulting in the formation of olivetolic acid. Sources: GOC:TermGenie Relationships: is a type of GO:0030639; is a type of benzene-containing compound metabolic process [GO:0042537]; is a type of phenol-containing compound biosynthetic process [GO:0046189]; is a type of monocarboxylic acid biosynthetic process [GO:0072330] Also known as: olivetolic acid anabolism, olivetolic acid biosynthesis, olivetolic acid formation, olivetolic acid synthesis